regulation of zygosporangium development [GO:0075272] (biological process) Sources: GOC:pamgo_curators Subtypes: positive regulation of zygosporangium development [GO:0075273], negative regulation of zygosporangium development [GO:0075274] Relationships: is a type of regulation of spore-bearing organ development [GO:0075260]; regulates GO:0075271 Definition: Any process that modulates the frequency, rate or extent of zygosporangium development, a process in which a fruiting body called zygosporangium is formed.